{
  "gene_name": "Protein lin-7 homolog C",
  "term_label": "neurotransmitter secretion",
  "term_id": "GO:0007269",
  "gene_symbol": "LIN7C",
  "gene": "UniProtKB:Q9NUP9"
}